{
  "term_label": "Unknown cellular component",
  "term_id": "UNKNOWN:0003",
  "gene_symbol": "ZNF763",
  "gene": "UniProtKB:Q0D2J5",
  "gene_name": "Zinc finger protein 763"
}